GABA-gated chloride ion channel activity [GO:0022851] (molecular function) Sources: GOC:mtg_transport, ISBN:0815340729 Relationships: is a type of chloride channel activity [GO:0005254]; is_a GO:0022824; is a type of ligand-gated monoatomic anion channel activity [GO:0099095] Definition: Enables the transmembrane transfer of a chloride ion by a channel that opens when GABA has been bound by the channel complex or one of its constituent parts.